{
  "term_label": "5'-3' exonuclease activity",
  "gene_symbol": "TRIR",
  "gene_name": "Telomerase RNA component interacting RNase",
  "gene": "UniProtKB:Q9BQ61",
  "term_id": "GO:0008409"
}